{
  "gene": "UniProtKB:Q3SYB3",
  "term_label": "Unknown cellular component",
  "gene_name": "Forkhead box protein D4-like 6",
  "term_id": "UNKNOWN:0003",
  "gene_symbol": "FOXD4L6"
}